{
  "term_id": "GO:0006357",
  "term_label": "regulation of transcription by RNA polymerase II",
  "gene_name": "Zinc finger protein 394",
  "gene": "UniProtKB:Q53GI3",
  "gene_symbol": "ZNF394"
}